{
  "term_id": "GO:0004430",
  "gene_name": "Phosphatidylinositol 4-kinase type 2-alpha",
  "term_label": "1-phosphatidylinositol 4-kinase activity",
  "gene": "UniProtKB:Q9BTU6",
  "gene_symbol": "PI4K2A"
}